{
  "gene_symbol": "PIMREG",
  "term_id": "UNKNOWN:0003",
  "term_label": "Unknown cellular component",
  "gene": "UniProtKB:Q9BSJ6",
  "gene_name": "Protein PIMREG"
}